{
  "term_id": "GO:0009897",
  "gene_symbol": "CXCR6",
  "gene": "UniProtKB:O00574",
  "term_label": "external side of plasma membrane",
  "gene_name": "C-X-C chemokine receptor type 6"
}